negative regulation of sevenless signaling pathway [GO:0045873] (BP) Definition: Any process that stops, prevents, or reduces the frequency, rate or extent of the sevenless signaling pathway. Sources: GOC:go_curators Also known as: down regulation of sevenless signaling pathway, down-regulation of sevenless signaling pathway, downregulation of sevenless signaling pathway, negative regulation of sev signaling pathway, negative regulation of sevenless signalling pathway, inhibition of sevenless signaling pathway Relationships: is a type of GO:0009968; is a type of negative regulation of cell fate commitment [GO:0010454]; is a type of GO:0045501; is a type of negative regulation of R7 cell differentiation [GO:0045677]; RO_0002212 sevenless signaling pathway [GO:0045500]